synaptic vesicle localization [GO:0097479] (biological process) Subtypes: synaptic vesicle transport [GO:0048489], synaptic vesicle clustering [GO:0097091] Relationships: is a type of vesicle localization [GO:0051648] Sources: GOC:pr Definition: Any process in which a synaptic vesicle or vesicles are transported to, and/or maintained in, a specific location. Also known as: establishment and maintenance of synaptic vesicle localization, establishment and maintenance of synaptic vesicle position, synaptic vesicle localisation